{
  "term_label": "Unknown biological process",
  "gene_name": "Sodium_myo-inositol cotransporter 2",
  "gene_symbol": "SLC5A11",
  "gene": "UniProtKB:Q8WWX8",
  "term_id": "UNKNOWN:0002"
}